aclacinomycin T methylesterase activity [GO:0102530] (molecular function) Relationships: is a type of carboxylic ester hydrolase activity [GO:0052689] Definition: Catalysis of the reaction: aclacinomycin T(1+) + H2O = 15-demethylaclacinomycin T + methanol + H+. Sources: EC:3.1.1.95, GOC:pz